{
  "gene": "UniProtKB:O75677",
  "term_id": "GO:0005737",
  "term_label": "cytoplasm",
  "gene_symbol": "RFPL1",
  "gene_name": "Ret finger protein-like 1"
}